{
  "gene_name": "Putative uncharacterized protein IBA57-DT",
  "term_label": "Unknown cellular component",
  "gene_symbol": "IBA57-DT",
  "term_id": "UNKNOWN:0003",
  "gene": "UniProtKB:B1ANH7"
}